{
  "term_id": "UNKNOWN:0001",
  "gene": "UniProtKB:Q9Y2H5",
  "gene_symbol": "PLEKHA6",
  "gene_name": "Pleckstrin homology domain-containing family A member 6",
  "term_label": "Unknown molecular function"
}